{
  "term_id": "GO:0015671",
  "gene_name": "Hemoglobin subunit theta-1",
  "gene_symbol": "HBQ1",
  "term_label": "oxygen transport",
  "gene": "UniProtKB:P09105"
}